regulation of interleukin-1 alpha production [GO:0032650] (biological process) Subtypes: negative regulation of interleukin-1 alpha production [GO:0032690], positive regulation of interleukin-1 alpha production [GO:0032730] Relationships: is a type of regulation of interleukin-1 production [GO:0032652]; regulates interleukin-1 alpha production [GO:0032610] Definition: Any process that modulates the frequency, rate, or extent of interleukin-1 alpha production. Sources: GOC:mah Also known as: regulation of IL-1 alpha production, regulation of interleukin-1 alpha biosynthetic process, regulation of interleukin-1 alpha secretion